presynaptic cytoskeleton organization [GO:0099187] (biological process) Definition: A process that is carried out at the cellular level which results in the assembly, arrangement of constituent parts, or disassembly of cytoskeletal structures and their associated proteins in the presynaptic cytoskeleton. Sources: GOC:dos Relationships: is a type of cytoskeleton organization [GO:0007010]; is part of GO:0099172 Subtypes: presynaptic actin cytoskeleton organization [GO:0099140]